{
  "term_label": "extracellular space",
  "gene_symbol": "TIMP3",
  "term_id": "GO:0005615",
  "gene_name": "Metalloproteinase inhibitor 3",
  "gene": "UniProtKB:P35625"
}